{
  "term_id": "GO:0009897",
  "gene_name": "Fc receptor-like B",
  "term_label": "external side of plasma membrane",
  "gene_symbol": "FCRLB",
  "gene": "UniProtKB:Q6BAA4"
}